{
  "term_id": "GO:0000380",
  "gene_name": "Probable ATP-dependent RNA helicase DDX5",
  "gene": "UniProtKB:P17844",
  "gene_symbol": "DDX5",
  "term_label": "alternative mRNA splicing, via spliceosome"
}